2',3'-cyclic GMP-AMP synthase activity [GO:0061501] (molecular function) Definition: Catalysis of the reaction: ATP + GTP = 2 diphosphate + cyclic G-P(2'-5')A-P(3'-5') (cyclic 2',3' GAMP). Relationships: is a type of cyclic GMP-AMP synthase activity [GO:0140699] Also known as: cyclic-GMP-AMP synthase activity, 2',3' cyclic GMP-AMP synthase activity, 2',3' cyclic-GMP-AMP synthase activity, cyclic 2',3' GAMP synthase activity References: PMID:23258413 Sources: GOC:dph, RHEA:42064